{
  "gene_symbol": "RRP12",
  "gene": "UniProtKB:Q5JTH9",
  "gene_name": "RRP12-like protein",
  "term_id": "GO:0003723",
  "term_label": "RNA binding"
}